innate immune response in mucosa [GO:0002227] (biological process) Definition: Any process of the innate immune response that takes place in the mucosal tissues. References: PMID:10719665, PMID:15971105 Sources: GOC:add Relationships: is_a GO:0002385; is a type of innate immune response [GO:0045087]